{
  "gene_name": "COP9 signalosome complex subunit 3",
  "gene_symbol": "COPS3",
  "term_label": "COP9 signalosome",
  "gene": "UniProtKB:Q9UNS2",
  "term_id": "GO:0008180"
}